{
  "gene_symbol": "SNRPE",
  "term_id": "GO:0046540",
  "gene_name": "Small nuclear ribonucleoprotein E",
  "term_label": "U4/U6 x U5 tri-snRNP complex",
  "gene": "UniProtKB:P62304"
}